deoxyribonuclease V activity [GO:0043737] (molecular function) Definition: Catalysis of the endonucleolytic cleavage at apurinic or apyrimidinic sites to products with a 5'-phosphate. Relationships: is a type of DNA endonuclease activity, producing 5'-phosphomonoesters [GO:0016888] Also known as: endonuclease V activity, endodeoxyribonuclease V, Escherichia coli endodeoxyribonuclease V activity, DNase V activity Sources: EC:3.1.21.7